{
  "gene": "UniProtKB:O14503",
  "gene_name": "Class E basic helix-loop-helix protein 40",
  "term_label": "regulation of neurogenesis",
  "term_id": "GO:0050767",
  "gene_symbol": "BHLHE40"
}